integrin biosynthetic process [GO:0045112] (biological process) Regulation: RO_0002211 by GO:0045113; negatively regulated by negative regulation of integrin biosynthetic process [GO:0045720]; positively regulated by GO:0045726 Subtypes: beta 2 integrin biosynthetic process [GO:0045114] Also known as: integrin anabolism, integrin biosynthesis, integrin formation, integrin synthesis Definition: The chemical reactions and pathways resulting in the formation of integrins, a large family of transmembrane proteins that act as receptors for cell-adhesion molecules. Sources: GOC:go_curators, ISBN:0198506732 Relationships: is_a macromolecule biosynthetic process [GO:0009059]; is part of plasma membrane organization [GO:0007009]